negative regulation of adaptive immune response based on somatic recombination of immune receptors built from immunoglobulin superfamily domains [GO:0002823] (biological process) Relationships: is a type of negative regulation of adaptive immune response [GO:0002820]; is a type of regulation of adaptive immune response based on somatic recombination of immune receptors built from immunoglobulin superfamily domains [GO:0002822]; negatively regulates adaptive immune response based on somatic recombination of immune receptors built from immunoglobulin superfamily domains [GO:0002460] Subtypes: negative regulation of germinal center formation [GO:0002635], negative regulation of tolerance induction dependent upon immune response [GO:0002653], negative regulation of T cell mediated immunity [GO:0002710], GO:0002713, GO:0002826, negative regulation of T-helper 17 type immune response [GO:2000317] Definition: Any process that stops, prevents, or reduces the frequency, rate, or extent of an adaptive immune response based on somatic recombination of immune receptors built from immunoglobulin superfamily domains. An example of this process is found in the Gnathostomata. Sources: GOC:add, GOC:mtg_sensu